{
  "gene_symbol": "CCDC18",
  "gene": "UniProtKB:Q5T9S5",
  "gene_name": "Coiled-coil domain-containing protein 18",
  "term_label": "Unknown molecular function",
  "term_id": "UNKNOWN:0001"
}